{
  "term_label": "ribonucleoside triphosphate phosphatase activity",
  "gene": "UniProtKB:Q9NQZ7",
  "term_id": "GO:0017111",
  "gene_name": "Ectonucleoside triphosphate diphosphohydrolase 7",
  "gene_symbol": "ENTPD7"
}